negative regulation of chemokine-mediated signaling pathway [GO:0070100] (biological process) Subtypes: negative regulation of C-C chemokine receptor CCR7 signaling pathway [GO:1903081] Sources: GOC:mah Also known as: negative regulation of chemokine-mediated signalling pathway Relationships: is a type of negative regulation of cytokine-mediated signaling pathway [GO:0001960]; is a type of negative regulation of G protein-coupled receptor signaling pathway [GO:0045744]; is a type of regulation of chemokine-mediated signaling pathway [GO:0070099]; RO_0002212 GO:0070098 Definition: Any process that decreases the rate, frequency or extent of a chemokine-mediated signaling pathway.